{
  "term_label": "chromatin",
  "gene": "UniProtKB:Q14103",
  "gene_symbol": "HNRNPD",
  "gene_name": "Heterogeneous nuclear ribonucleoprotein D0",
  "term_id": "GO:0000785"
}